{
  "gene_name": "Uncharacterized protein C2orf15",
  "term_label": "Unknown molecular function",
  "term_id": "UNKNOWN:0001",
  "gene": "UniProtKB:Q8WU43",
  "gene_symbol": "C2orf15"
}